{
  "term_label": "Golgi organization",
  "gene_symbol": "COG3",
  "term_id": "GO:0007030",
  "gene_name": "Conserved oligomeric Golgi complex subunit 3",
  "gene": "UniProtKB:Q96JB2"
}